{
  "gene_symbol": "POTEKP",
  "term_id": "GO:0015629",
  "term_label": "actin cytoskeleton",
  "gene_name": "Putative beta-actin-like protein 3",
  "gene": "UniProtKB:Q9BYX7"
}